potassium:chloride symporter activity [GO:0015379] (molecular function) Subtypes: GO:0008511 Relationships: is a type of GO:0015079; is_a chloride:monoatomic cation symporter activity [GO:0015377] Also known as: potassium ion symporter activity Definition: Enables the transfer of a solute or solutes from one side of a membrane to the other according to the reaction: K+(out) + Cl-(out) = K+(in) + Cl-(in). Sources: TC:2.A.30.1.5